{
  "term_label": "fatty acid catabolic process",
  "gene": "UniProtKB:Q6ZUV0",
  "gene_name": "Putative cytosolic acyl coenzyme A thioester hydrolase-like",
  "gene_symbol": "ACOT7L",
  "term_id": "GO:0009062"
}